{
  "gene": "UniProtKB:Q7Z7M9",
  "gene_symbol": "GALNT5",
  "term_label": "polypeptide N-acetylgalactosaminyltransferase activity",
  "gene_name": "Polypeptide N-acetylgalactosaminyltransferase 5",
  "term_id": "GO:0004653"
}